ascospore wall beta-glucan metabolic process [GO:0034408] (biological process) Relationships: is a type of fungal-type cell wall beta-glucan metabolic process [GO:0070879]; is a type of meiotic cell cycle process [GO:1903046]; is part of GO:0070591 Definition: The chemical reactions and pathways involving beta-glucans, compounds composed of glucose residues linked by beta-D-glucosidic bonds, found in the walls of ascospores. Subtypes: GO:0034409, ascospore wall beta-glucan biosynthetic process [GO:0034412] Also known as: ascospore wall beta-glucan metabolism Sources: GOC:mah